{
  "gene_name": "2-iminobutanoate_2-iminopropanoate deaminase",
  "term_label": "cytosol",
  "gene": "UniProtKB:P52758",
  "term_id": "GO:0005829",
  "gene_symbol": "RIDA"
}